{
  "term_label": "chromosome condensation",
  "term_id": "GO:0030261",
  "gene": "UniProtKB:P16402",
  "gene_symbol": "H1-3",
  "gene_name": "Histone H1.3"
}